{
  "gene_symbol": "TOPORS",
  "term_label": "protein monoubiquitination",
  "gene": "UniProtKB:Q9NS56",
  "term_id": "GO:0006513",
  "gene_name": "E3 ubiquitin-protein ligase Topors"
}